meiotic prophase I [GO:0007128] (biological process) Note: Note that this term should not be used for direct annotation. If you are trying to make an annotation to x phase, it is likely that the correct annotation is 'regulation of x/y phase transition' or to a process which occurs during the reported phase (i.e mitotic DNA replication for mitotic S-phase). To capture the phase when a specific location or process is observed, the phase term can be used in an annotation extension (PMID:24885854) applied to a cellular component term (with the relation exists_during) or a biological process term (with the relation happens_during). Definition: The cell cycle phase which is the first stage of meiosis I and during which chromosomes condense and the two daughter centrioles and their asters migrate toward the poles of the cell. Sources: GOC:mtg_cell_cycle Relationships: is a type of prophase [GO:0051324]; is a type of meiosis I cell cycle phase [GO:0098764]